{
  "term_label": "neuron projection development",
  "term_id": "GO:0031175",
  "gene_symbol": "FRYL",
  "gene_name": "Protein furry homolog-like",
  "gene": "UniProtKB:O94915"
}